{
  "gene_name": "Tyrosine-protein kinase Srms",
  "gene_symbol": "SRMS",
  "term_label": "cell differentiation",
  "gene": "UniProtKB:Q9H3Y6",
  "term_id": "GO:0030154"
}